{
  "term_label": "proteasome-mediated ubiquitin-dependent protein catabolic process",
  "gene_name": "26S proteasome regulatory subunit 4",
  "gene": "UniProtKB:P62191",
  "term_id": "GO:0043161",
  "gene_symbol": "PSMC1"
}